{
  "gene_symbol": "BLNK",
  "term_label": "B cell receptor signaling pathway",
  "term_id": "GO:0050853",
  "gene_name": "B-cell linker protein",
  "gene": "UniProtKB:Q8WV28"
}